{
  "gene_name": "Protein unc-119 homolog B",
  "term_label": "lipoprotein transport",
  "gene": "UniProtKB:A6NIH7",
  "gene_symbol": "UNC119B",
  "term_id": "GO:0042953"
}